{
  "gene": "UniProtKB:Q14028",
  "term_id": "GO:0098655",
  "term_label": "monoatomic cation transmembrane transport",
  "gene_name": "Cyclic nucleotide-gated cation channel beta-1",
  "gene_symbol": "CNGB1"
}